{
  "gene_name": "Brain-specific homeobox protein homolog",
  "gene": "UniProtKB:Q3C1V8",
  "term_id": "GO:0030154",
  "term_label": "cell differentiation",
  "gene_symbol": "BSX"
}